MHC class Ib receptor activity [GO:0032394] (molecular function) Definition: Combining with an MHC class Ib protein complex and transmitting the signal from one side of the membrane to the other to initiate a change in cell activity. Class Ib here refers to non-classical class I molecules, such as those of the CD1 or HLA-E gene families. Sources: GOC:add, GOC:signaling, ISBN:0781735149 Subtypes: inhibitory MHC class Ib receptor activity [GO:0062080], activating MHC class Ib receptor activity [GO:0062081] Note: Note that this term is intended for annotation of gene products that act as receptors for MHC class Ib protein complexes, not for components of the MHC class Ib protein complexes themselves. Also known as: T cell receptor activity, alpha-beta T cell receptor activity, gamma-delta T cell receptor activity Relationships: is a type of transmembrane signaling receptor activity [GO:0004888]; is a type of GO:0140375; has part MHC class Ib protein binding [GO:0023029]